regulation of saliva secretion [GO:0046877] (biological process) Definition: Any process that modulates the frequency, rate or extent of the regulated release of saliva from a cell or a tissue. Relationships: is a type of regulation of digestive system process [GO:0044058]; is a type of GO:0050878; is a type of regulation of secretion [GO:0051046]; regulates GO:0046541 Subtypes: GO:0046878, negative regulation of saliva secretion [GO:1905747] Sources: GOC:ai